positive regulation of protein sumoylation [GO:0033235] (biological process) Sources: GOC:mah Also known as: positive regulation of sumoylation Relationships: is_a regulation of protein sumoylation [GO:0033233]; is a type of positive regulation of protein modification by small protein conjugation or removal [GO:1903322]; positively regulates protein sumoylation [GO:0016925] Definition: Any process that activates or increases the frequency, rate or extent of the addition of SUMO groups to a protein.